succinate transport [GO:0015744] (BP) Relationships: is a type of C4-dicarboxylate transport [GO:0015740] Sources: GOC:krc Definition: The directed movement of succinate, the dianion of ethane dicarboxylic acid, into, out of or within a cell, or between cells, by means of some agent such as a transporter or pore. Subtypes: succinate transmembrane transport [GO:0071422]